{
  "gene_name": "Glutamate receptor 2",
  "term_label": "transmitter-gated monoatomic ion channel activity involved in regulation of postsynaptic membrane potential",
  "gene_symbol": "GRIA2",
  "gene": "UniProtKB:P42262",
  "term_id": "GO:1904315"
}